{
  "term_label": "apolipoprotein binding",
  "gene_name": "Prolow-density lipoprotein receptor-related protein 1",
  "term_id": "GO:0034185",
  "gene_symbol": "LRP1",
  "gene": "UniProtKB:Q07954"
}